FACIT collagen trimer [GO:0005593] (CC) Subtypes: collagen type IX trimer [GO:0005594], GO:0005595, collagen type XIV trimer [GO:0005596], collagen type XVI trimer [GO:0005597], GO:1990319, collagen type XXI trimer [GO:1990320], collagen type XXII trimer [GO:1990321] Note: The acronym FACIT stands for fibril-associated collagen with interrupted triple helix. Definition: A collagen trimer that associates with collagen fibrils and consists of collagen monomers that contain two or more relatively short triple-helical domains connected by non-triple-helical sequences. References: PMID:21421911 Relationships: is a type of collagen trimer [GO:0005581]; is part of FACIT collagen complex [GO:0140153]